amino acid conjugated cholate hydrolase activity [GO:7770003] (molecular function) References: PMID:38326608, PMID:38326609, PMID:40446798 Sources: RHEA:79087 Definition: Catalysis of the reaction: an L-alpha-amino acid + cholate = an N-choloyl-L-alpha-amino acid + H2O. Relationships: is a type of hydrolase activity, acting on carbon-nitrogen (but not peptide) bonds, in linear amides [GO:0016811] Subtypes: L-serine conjugated cholate hydrolase activity [GO:7770004], L-alanine conjugated cholate hydrolase activity [GO:7770005], L-phenylalanine conjugated cholate hydrolase activity [GO:7770006], GO:7770007, L-histidine conjugated cholate hydrolase activity [GO:7770008], L-tryptophan conjugated cholate hydrolase activity [GO:7770009]